{
  "gene": "UniProtKB:Q14831",
  "term_id": "GO:0005886",
  "term_label": "plasma membrane",
  "gene_symbol": "GRM7",
  "gene_name": "Metabotropic glutamate receptor 7"
}